{
  "gene": "UniProtKB:P01763",
  "gene_name": "Immunoglobulin heavy variable 3-48",
  "term_id": "GO:0016064",
  "term_label": "immunoglobulin mediated immune response",
  "gene_symbol": "IGHV3-48"
}